{
  "gene_symbol": "GNAZ",
  "term_id": "GO:0005737",
  "gene": "UniProtKB:P19086",
  "term_label": "cytoplasm",
  "gene_name": "Guanine nucleotide-binding protein G(z) subunit alpha"
}